{
  "gene_name": "Olfactory receptor 5C1",
  "gene": "UniProtKB:Q8NGR4",
  "gene_symbol": "OR5C1",
  "term_label": "Unknown cellular component",
  "term_id": "UNKNOWN:0003"
}